dehiscence [GO:0009900] (biological process) Sources: ISBN:0879015322 Subtypes: anther dehiscence [GO:0009901], GO:0010047 Definition: The opening of an anther, fruit or other structure, which permits the escape of reproductive bodies contained within it. Relationships: is a type of GO:0048609